{
  "term_label": "positive regulation of cell-substrate adhesion",
  "gene_symbol": "FBLN2",
  "term_id": "GO:0010811",
  "gene_name": "Fibulin-2",
  "gene": "UniProtKB:P98095"
}